{
  "gene_name": "Gem-associated protein 7",
  "term_id": "GO:0120114",
  "term_label": "Sm-like protein family complex",
  "gene": "UniProtKB:Q9H840",
  "gene_symbol": "GEMIN7"
}